{
  "term_id": "GO:0016323",
  "gene": "UniProtKB:P21730",
  "gene_symbol": "C5AR1",
  "term_label": "basolateral plasma membrane",
  "gene_name": "C5a anaphylatoxin chemotactic receptor 1"
}